{
  "gene_symbol": "BOK",
  "term_label": "positive regulation of apoptotic process",
  "term_id": "GO:0043065",
  "gene_name": "Bcl-2-related ovarian killer protein",
  "gene": "UniProtKB:Q9UMX3"
}